{
  "gene_name": "Sodium_potassium_calcium exchanger 2",
  "gene_symbol": "SLC24A2",
  "term_id": "GO:0005886",
  "term_label": "plasma membrane",
  "gene": "UniProtKB:Q9UI40"
}